{
  "gene": "UniProtKB:Q13188",
  "term_id": "GO:0090090",
  "gene_symbol": "STK3",
  "gene_name": "Serine_threonine-protein kinase 3",
  "term_label": "negative regulation of canonical Wnt signaling pathway"
}